{
  "gene_name": "Death-associated protein-like 1",
  "term_label": "apoptotic signaling pathway",
  "gene": "UniProtKB:A0PJW8",
  "gene_symbol": "DAPL1",
  "term_id": "GO:0097190"
}